{
  "term_id": "GO:0043418",
  "gene": "UniProtKB:Q13867",
  "gene_name": "Bleomycin hydrolase",
  "gene_symbol": "BLMH",
  "term_label": "homocysteine catabolic process"
}